inactivation of recombination (HML) [GO:0007537] (biological process) Definition: The inactivation of recombination at sequences around a mating type donor locus, with the consequence that the other donor is the only one available for mating type switching; exemplified by the HML locus and surrounding sequences on Chromosome III in Saccharomyces cerevisiae. References: PMID:9928492 Sources: GOC:mah Relationships: is_a donor selection [GO:0007535]; is a type of GO:0045910